{
  "gene_name": "BMP_retinoic acid-inducible neural-specific protein 1",
  "gene": "UniProtKB:O60477",
  "term_id": "GO:0021953",
  "gene_symbol": "BRINP1",
  "term_label": "central nervous system neuron differentiation"
}